{
  "gene": "UniProtKB:Q5JZY3",
  "gene_symbol": "EPHA10",
  "term_id": "GO:0005005",
  "term_label": "transmembrane-ephrin receptor activity",
  "gene_name": "Ephrin type-A receptor 10"
}